formin-nucleated actin cable assembly [GO:0070649] (biological process) Also known as: formin-nucleated actin cable formation References: PMID:14671023, PMID:16959963 Sources: GOC:mah Definition: The aggregation, arrangement and bonding together of a set of components to form a formin-nucleated actin cable. A formin-nucleated actin cable is an actin filament bundle that consists of short filaments organized into bundles of uniform polarity, and is nucleated by formins. Regulation: regulated by GO:0090337; positively regulated by positive regulation of formin-nucleated actin cable assembly [GO:0090338]; negatively regulated by GO:0090339 Relationships: is a type of parallel actin filament bundle assembly [GO:0030046]; is_a formin-nucleated actin cable organization [GO:0110009]